{
  "gene_symbol": "AP1G1",
  "term_label": "AP-1 adaptor complex",
  "gene": "UniProtKB:O43747",
  "term_id": "GO:0030121",
  "gene_name": "AP-1 complex subunit gamma-1"
}